{
  "gene_symbol": "SPEF2",
  "term_label": "sperm midpiece",
  "term_id": "GO:0097225",
  "gene": "UniProtKB:Q9C093",
  "gene_name": "Sperm flagellar protein 2"
}